{
  "gene_symbol": "ZNF503",
  "gene_name": "Zinc finger protein 503",
  "term_label": "nucleus",
  "term_id": "GO:0005634",
  "gene": "UniProtKB:Q96F45"
}